{
  "term_id": "UNKNOWN:0003",
  "gene": "UniProtKB:P02771",
  "term_label": "Unknown cellular component",
  "gene_symbol": "AFP",
  "gene_name": "Alpha-fetoprotein"
}